{
  "term_label": "plasma membrane",
  "term_id": "GO:0005886",
  "gene": "UniProtKB:O75955",
  "gene_symbol": "FLOT1",
  "gene_name": "Flotillin-1"
}